{
  "term_id": "GO:0005829",
  "gene_symbol": "NMT2",
  "gene": "UniProtKB:O60551",
  "term_label": "cytosol",
  "gene_name": "Glycylpeptide N-tetradecanoyltransferase 2"
}